AMP transmembrane transporter activity [GO:0080122] (molecular function) Definition: Enables the transfer of AMP, adenosine monophosphate, from one side of a membrane to the other. Also known as: adenosine monophosphate transmembrane transporter activity Relationships: is a type of adenine nucleotide transmembrane transporter activity [GO:0000295]; is a type of purine ribonucleotide transmembrane transporter activity [GO:0005346]; is part of GO:0080121 References: PMID:18923018